{
  "gene_symbol": "RGPD5",
  "term_id": "GO:0005643",
  "gene": "UniProtKB:Q99666",
  "gene_name": "RANBP2-like and GRIP domain-containing protein 5_6",
  "term_label": "nuclear pore"
}